{
  "gene_symbol": "CXCL16",
  "term_label": "scavenger receptor activity",
  "term_id": "GO:0005044",
  "gene": "UniProtKB:Q9H2A7",
  "gene_name": "C-X-C motif chemokine 16"
}